{
  "gene_symbol": "PNMA6A",
  "term_id": "UNKNOWN:0001",
  "gene_name": "Paraneoplastic antigen-like protein 6A",
  "gene": "UniProtKB:P0CW24",
  "term_label": "Unknown molecular function"
}